type I interferon production [GO:0032606] (biological process) Relationships: is a type of cytokine production [GO:0001816] Note: Note that this term is in the subset of terms that should not be used for direct gene product annotation. Instead, select one of the 'regulation' children terms. Also known as: interferon type I production, type I IFN production, type I interferon biosynthetic process, type I interferon secretion Regulation: RO_0002211 by regulation of type I interferon production [GO:0032479]; negatively regulated by negative regulation of type I interferon production [GO:0032480]; positively regulated by positive regulation of type I interferon production [GO:0032481] References: PMID:15546383, PMID:16681834 Sources: GOC:add, ISBN:0126896631 Definition: The appearance of type I interferon due to biosynthesis or secretion following a cellular stimulus, resulting in an increase in its intracellular or extracellular levels. Type I interferons include the interferon-alpha, beta, delta, episilon, zeta, kappa, tau, and omega gene families. Subtypes: GO:0032607, GO:0032608, interferon-delta production [GO:0072645], GO:0072647, interferon-kappa production [GO:0072649], GO:0072651, interferon-omega production [GO:0072653]